{
  "gene_symbol": "CYP26C1",
  "term_id": "GO:0007417",
  "gene_name": "Cytochrome P450 26C1",
  "gene": "UniProtKB:Q6V0L0",
  "term_label": "central nervous system development"
}